{
  "gene_name": "Uncharacterized protein",
  "term_id": "UNKNOWN:0003",
  "gene_symbol": "LOC122526780",
  "term_label": "Unknown cellular component",
  "gene": "UniProtKB:A0A590UJ96"
}